{
  "gene_name": "Zinc finger E-box-binding homeobox 1",
  "term_label": "RNA polymerase II cis-regulatory region sequence-specific DNA binding",
  "gene": "UniProtKB:P37275",
  "gene_symbol": "ZEB1",
  "term_id": "GO:0000978"
}